peptidyl-pyrromethane cofactor linkage [GO:0018160] (biological process) Relationships: is a type of peptidyl-cysteine modification [GO:0018198] Definition: The covalent binding of a pyrromethane (dipyrrin) cofactor to protein via the sulfur atom of cysteine forming dipyrrolylmethanemethyl-L-cysteine. Sources: RESID:AA0252 Also known as: peptidyl-pyrromethane cofactor linkage via dipyrrolylmethanemethyl-L-cysteine, dipyrromethane cofactor binding